tricarboxylic acid transmembrane transport [GO:0035674] (biological process) Subtypes: GO:1990546 Sources: GOC:vw Also known as: tricarboxylic acid membrane transport Definition: The process in which a tricarboxylic acid is transported across a membrane. Relationships: is a type of carboxylic acid transmembrane transport [GO:1905039] Note: Note that this term is not intended for use in annotating lateral movement within membranes.